mitotic spindle pole body organization [GO:1905047] (biological process) Definition: A process that is carried out at the cellular level which results in the assembly, arrangement of constituent parts, or disassembly of a mitotic spindle pole body. References: PMID:24963130 Sources: GOC:TermGenie Relationships: is a type of GO:0051300